{
  "gene_symbol": "IFI27L2",
  "gene_name": "Interferon alpha-inducible protein 27-like protein 2",
  "gene": "UniProtKB:Q9H2X8",
  "term_id": "GO:0031966",
  "term_label": "mitochondrial membrane"
}